{
  "gene_name": "Insulin-like growth factor-binding protein 3",
  "gene_symbol": "IGFBP3",
  "term_label": "fibronectin binding",
  "gene": "UniProtKB:P17936",
  "term_id": "GO:0001968"
}